{
  "gene_name": "Orexin receptor type 2",
  "gene": "UniProtKB:O43614",
  "term_id": "GO:0007218",
  "term_label": "neuropeptide signaling pathway",
  "gene_symbol": "HCRTR2"
}